{
  "gene_symbol": "SEMA3B",
  "gene": "UniProtKB:Q13214",
  "gene_name": "Semaphorin-3B",
  "term_id": "GO:0045499",
  "term_label": "chemorepellent activity"
}